{
  "term_id": "GO:0007214",
  "gene_symbol": "GPR156",
  "gene_name": "Probable G-protein coupled receptor 156",
  "term_label": "gamma-aminobutyric acid signaling pathway",
  "gene": "UniProtKB:Q8NFN8"
}